sodium:chloride symporter activity [GO:0015378] (molecular function) Relationships: is a type of monoatomic anion:sodium symporter activity [GO:0015373]; is_a GO:0015377 Subtypes: dopamine:sodium symporter activity [GO:0005330], gamma-aminobutyric acid:sodium:chloride symporter activity [GO:0005332], norepinephrine:sodium symporter activity [GO:0005334], serotonin:sodium:chloride symporter activity [GO:0005335], sodium:potassium:chloride symporter activity [GO:0008511], glycine betaine:sodium:chloride symporter activity [GO:0140814], neutral L-amino acid:sodium:chloride symporter activity [GO:0140931], sodium:ammonium:chloride symporter activity [GO:7770002] Sources: TC:2.A.30.4.- Definition: Enables the transfer of a solute or solutes from one side of a membrane to the other according to the reaction: Na+(out) + Cl-(out) = Na+(in) + Cl-(in).